{
  "term_label": "regulation of transcription by RNA polymerase II",
  "gene": "UniProtKB:Q9ULD4",
  "gene_symbol": "BRPF3",
  "term_id": "GO:0006357",
  "gene_name": "Bromodomain and PHD finger-containing protein 3"
}